ACU codon-amino acid adaptor activity [GO:0033437] (molecular function) Also known as: ACT codon-amino acid adaptor activity, threonine tRNA Relationships: is a type of triplet codon-amino acid adaptor activity [GO:0030533] Note: Note that in the standard genetic code, ACT codes for threonine. Sources: GOC:mah Definition: A triplet codon-amino acid adaptor activity that recognizes an ACU codon.